{
  "term_id": "GO:0005634",
  "term_label": "nucleus",
  "gene_symbol": "PASK",
  "gene_name": "PAS domain-containing serine_threonine-protein kinase",
  "gene": "UniProtKB:Q96RG2"
}